{
  "gene_name": "Nebulette",
  "term_label": "cardiac muscle thin filament assembly",
  "term_id": "GO:0071691",
  "gene": "UniProtKB:O76041",
  "gene_symbol": "NEBL"
}